{
  "gene_symbol": "TFDP2",
  "gene_name": "Transcription factor Dp-2",
  "gene": "UniProtKB:Q14188",
  "term_label": "RNA polymerase II transcription regulatory region sequence-specific DNA binding",
  "term_id": "GO:0000977"
}